{
  "term_id": "GO:0006357",
  "gene_symbol": "ZNF684",
  "gene_name": "Zinc finger protein 684",
  "gene": "UniProtKB:Q5T5D7",
  "term_label": "regulation of transcription by RNA polymerase II"
}